proline transport [GO:0015824] (biological process) Relationships: is a type of organic cation transport [GO:0015695]; is a type of neutral amino acid transport [GO:0015804]; is_a L-amino acid transport [GO:0015807] Sources: GOC:ai Regulation: regulated by regulation of proline transport [GO:0070881] Definition: The directed movement of proline, pyrrolidine-2-carboxylic acid, into, out of or within a cell, or between cells, by means of some agent such as a transporter or pore. Also known as: L-proline transport Subtypes: L-proline transmembrane transport [GO:1904555]